GUG codon-amino acid adaptor activity [GO:0033452] (molecular function) Also known as: GTG codon-amino acid adaptor activity, valine tRNA Relationships: is a type of GO:0030533 Sources: GOC:mah Note: Note that in the standard genetic code, GTG codes for valine. Definition: A triplet codon-amino acid adaptor activity that recognizes a GUG codon.